establishment of planar polarity of follicular epithelium [GO:0042247] (biological process) Definition: Coordinated organization of groups of cells in the plane of a follicular epithelium, such that they all orient to similar coordinates. Relationships: is a type of establishment of planar polarity [GO:0001736]; is a type of establishment or maintenance of polarity of follicular epithelium [GO:0016334] Sources: GOC:ascb_2009, GOC:bf, GOC:dph, GOC:tb